{
  "term_id": "GO:0005741",
  "gene": "UniProtKB:Q9BWH2",
  "gene_name": "FUN14 domain-containing protein 2",
  "term_label": "mitochondrial outer membrane",
  "gene_symbol": "FUNDC2"
}